acidocalcisome [GO:0020022] (CC) Sources: GOC:mb Also known as: metachromatic granule, volutin granule, polyphosphate vacuole Relationships: is a type of intracellular membrane-bounded organelle [GO:0043231]; is part of GO:0005737 Definition: An electron-dense acidic membrane-bounded organelle which contains a matrix of pyrophosphate and polyphosphates with bound calcium and other cations.